{
  "term_id": "UNKNOWN:0002",
  "gene_name": "Putative uncharacterized protein B3GALT5-AS1",
  "gene_symbol": "B3GALT5-AS1",
  "term_label": "Unknown biological process",
  "gene": "UniProtKB:P59052"
}